{
  "gene_symbol": "ABITRAM",
  "term_label": "dendrite",
  "term_id": "GO:0030425",
  "gene_name": "Protein Abitram",
  "gene": "UniProtKB:Q9NX38"
}